{
  "gene_name": "Type I iodothyronine deiodinase",
  "term_id": "GO:0042403",
  "term_label": "thyroid hormone metabolic process",
  "gene_symbol": "DIO1",
  "gene": "UniProtKB:P49895"
}